{
  "gene": "UniProtKB:P02760",
  "term_label": "serine-type endopeptidase inhibitor activity",
  "gene_name": "Protein AMBP",
  "gene_symbol": "AMBP",
  "term_id": "GO:0004867"
}